{
  "term_id": "GO:0005737",
  "term_label": "cytoplasm",
  "gene_name": "Dedicator of cytokinesis protein 2",
  "gene_symbol": "DOCK2",
  "gene": "UniProtKB:Q92608"
}